response to brassinosteroid [GO:0009741] (BP) Definition: Any process that results in a change in state or activity of a cell or an organism (in terms of movement, secretion, enzyme production, gene expression, etc.) as a result of a brassinosteroid stimulus. Also known as: response to brassinosteroid stimulus Sources: GOC:jl Subtypes: GO:0009729, cellular response to brassinosteroid stimulus [GO:0071367] Relationships: is a type of GO:0009725; is a type of response to lipid [GO:0033993]; is a type of response to oxygen-containing compound [GO:1901700]